{
  "gene_symbol": "TADA2A",
  "gene_name": "Transcriptional adapter 2-alpha",
  "gene": "UniProtKB:O75478",
  "term_label": "transcription coactivator activity",
  "term_id": "GO:0003713"
}